{
  "term_id": "GO:0007186",
  "gene_symbol": "GPR174",
  "gene_name": "Probable G-protein coupled receptor 174",
  "term_label": "G protein-coupled receptor signaling pathway",
  "gene": "UniProtKB:Q9BXC1"
}